{
  "term_label": "synapse",
  "gene_symbol": "AGRN",
  "gene": "UniProtKB:O00468",
  "term_id": "GO:0045202",
  "gene_name": "Agrin"
}